{
  "gene_symbol": "GNG2",
  "gene_name": "Guanine nucleotide-binding protein G(I)_G(S)_G(O) subunit gamma-2",
  "term_id": "GO:0007186",
  "gene": "UniProtKB:P59768",
  "term_label": "G protein-coupled receptor signaling pathway"
}